{
  "term_id": "GO:0030496",
  "gene_name": "Centrosomal protein of 55 kDa",
  "term_label": "midbody",
  "gene": "UniProtKB:Q53EZ4",
  "gene_symbol": "CEP55"
}